acetylcholine-mediated vasodilation involved in regulation of systemic arterial blood pressure [GO:0003069] (biological process) Definition: The process in which acetylcholine signaling causes vasodilation, resulting in a change in blood pressure. Sources: GOC:mtg_cardio, GOC:rl Also known as: vasodilation by acetylcholine involved in regulation of systemic arterial blood pressure Relationships: is a type of negative regulation of systemic arterial blood pressure [GO:0003085]; is a type of vasodilation [GO:0042311]; is part of regulation of systemic arterial blood pressure by acetylcholine [GO:0003068]